{
  "term_id": "GO:0005183",
  "term_label": "gonadotropin hormone-releasing hormone activity",
  "gene_name": "Progonadoliberin-2",
  "gene": "UniProtKB:O43555",
  "gene_symbol": "GNRH2"
}